{
  "term_id": "UNKNOWN:0003",
  "gene": "UniProtKB:Q9UNW8",
  "gene_name": "Probable G-protein coupled receptor 132",
  "gene_symbol": "GPR132",
  "term_label": "Unknown cellular component"
}